UDP-glucose 6-dehydrogenase activity [GO:0003979] (MF) Definition: Catalysis of the reaction: H2O + 2 NAD+ + UDP-alpha-D-glucose = 3 H+ + 2 NADH + UDP-alpha-D-glucuronate. Relationships: is_a oxidoreductase activity, acting on the CH-OH group of donors, NAD or NADP as acceptor [GO:0016616] Sources: EC:1.1.1.22, RHEA:23596